{
  "gene_symbol": "PPIE",
  "gene": "UniProtKB:Q9UNP9",
  "term_label": "catalytic step 2 spliceosome",
  "term_id": "GO:0071013",
  "gene_name": "Peptidyl-prolyl cis-trans isomerase E"
}